{
  "term_label": "Unknown molecular function",
  "gene_symbol": "CCDC166",
  "gene": "UniProtKB:P0CW27",
  "term_id": "UNKNOWN:0001",
  "gene_name": "Coiled-coil domain-containing protein 166"
}